negative regulation of chromosome separation [GO:1905819] (biological process) Subtypes: negative regulation of meiotic chromosome separation [GO:1905133], negative regulation of mitotic sister chromatid separation [GO:2000816] References: PMID:21795393 Sources: GOC:TermGenie, GOC:bhm, GO_REF:0000058 Also known as: down regulation of chromosome separation, down-regulation of chromosome separation, downregulation of chromosome separation, down regulation of rDNA separation, down-regulation of rDNA separation, downregulation of rDNA separation, inhibition of chromosome separation, inhibition of rDNA separation, negative regulation of rDNA separation, down regulation of chromatid release, down-regulation of chromatid release, downregulation of chromatid release, inhibition of chromatid release, negative regulation of chromatid release Relationships: is a type of GO:0051985; is a type of regulation of chromosome separation [GO:1905818]; negatively regulates GO:0051304 Definition: Any process that stops, prevents or reduces the frequency, rate or extent of chromosome separation.